IscS-IscU complex [GO:1990330] (CC) References: PMID:20404999 Sources: GOC:bhm Relationships: is a type of GO:1990221; is a type of iron-sulfur cluster assembly complex [GO:1990229] Definition: A heterotetrameric protein complex involved in the sulfur transfer during iron-sulfur cluster assembly and in the modification of tRNA wobble positions. In E. coli it consists of a central IscS dimer with the IscU protomers attached to one of the IscS units each via a disulfide (-SSH) group.